myoblast differentiation [GO:0045445] (biological process) Subtypes: myoblast differentiation involved in skeletal muscle regeneration [GO:0014835], GO:0060379 Also known as: myoblast cell differentiation Regulation: regulated by regulation of myoblast differentiation [GO:0045661]; negatively regulated by negative regulation of myoblast differentiation [GO:0045662]; positively regulated by positive regulation of myoblast differentiation [GO:0045663] Definition: The process in which a relatively unspecialized cell acquires specialized features of a myoblast. A myoblast is a mononucleate cell type that, by fusion with other myoblasts, gives rise to the myotubes that eventually develop into striated muscle fibers. Sources: CL:0000056, GOC:go_curators, GOC:mtg_muscle Relationships: is a type of cell differentiation [GO:0030154]; is part of muscle structure development [GO:0061061]